{
  "gene": "UniProtKB:Q9Y6G1",
  "gene_symbol": "TMEM14A",
  "term_id": "GO:0031966",
  "gene_name": "Transmembrane protein 14A",
  "term_label": "mitochondrial membrane"
}